ciliary plasm [GO:0097014] (cellular component) Relationships: is a type of GO:0032838; is part of cilium [GO:0005929] Note: Note that we deem cilium and microtubule-based flagellum to be equivalent. Also, researchers consider the composition of both the plasm and the membrane of the cilium to be detectably different from that in the non-ciliary cytosol and plasma membrane (e.g. in terms of calcium ion concentration, membrane lipid composition, and more). For this reason, the term "ciliary plasm" is not linked to "cytoplasm". Also known as: cilium plasm, microtubule-based flagellar matrix, microtubule-based flagellum matrix, cilial cytoplasm, ciliary cytoplasm, cilium cytoplasm, microtubule-based flagellar cytoplasm, microtubule-based flagellum cytoplasm References: PMID:17895364 Sources: GOC:BHF, GOC:cilia, GOC:dos Definition: All of the contents of a cilium, excluding the plasma membrane surrounding the cilium.